{
  "gene_name": "HUWE1-associated protein modifying stress responses 2",
  "term_id": "UNKNOWN:0003",
  "gene_symbol": "HAPSTR2",
  "term_label": "Unknown cellular component",
  "gene": "UniProtKB:A0A7P0TBJ1"
}